{
  "term_id": "GO:0004867",
  "term_label": "serine-type endopeptidase inhibitor activity",
  "gene_symbol": "SPINK14",
  "gene": "UniProtKB:Q6IE38",
  "gene_name": "Serine protease inhibitor Kazal-type 14"
}